{
  "gene_symbol": "CPQ",
  "gene": "UniProtKB:Q9Y646",
  "term_id": "GO:0043171",
  "gene_name": "Carboxypeptidase Q",
  "term_label": "peptide catabolic process"
}